{
  "term_id": "UNKNOWN:0002",
  "gene": "UniProtKB:Q9H6L4",
  "term_label": "Unknown biological process",
  "gene_name": "Armadillo repeat-containing protein 7",
  "gene_symbol": "ARMC7"
}